{
  "term_id": "GO:0000981",
  "gene_name": "Max-interacting protein 1",
  "gene_symbol": "MXI1",
  "term_label": "DNA-binding transcription factor activity, RNA polymerase II-specific",
  "gene": "UniProtKB:P50539"
}